{
  "gene_symbol": "ABHD10",
  "gene": "UniProtKB:Q9NUJ1",
  "gene_name": "Palmitoyl-protein thioesterase ABHD10, mitochondrial",
  "term_label": "hydrolase activity, hydrolyzing O-glycosyl compounds",
  "term_id": "GO:0004553"
}